{
  "gene": "UniProtKB:Q8WWT9",
  "term_label": "citrate transmembrane transporter activity",
  "gene_name": "Na(+)_dicarboxylate cotransporter 3",
  "term_id": "GO:0015137",
  "gene_symbol": "SLC13A3"
}